'de novo' IMP biosynthetic process [GO:0006189] (biological process) Definition: The chemical reactions and pathways resulting in the formation of IMP, inosine monophosphate, by the stepwise assembly of a purine ring on ribose 5-phosphate. Sources: GOC:mah, ISBN:0716720094 Also known as: 'de novo' purine biosynthesis, 'de novo' purine biosynthetic process, 'de novo' IMP anabolism, 'de novo' IMP biosynthesis, 'de novo' IMP formation, 'de novo' IMP synthesis Relationships: is_a IMP biosynthetic process [GO:0006188]